{
  "gene_symbol": "PNPLA7",
  "term_id": "GO:0004622",
  "term_label": "phosphatidylcholine lysophospholipase activity",
  "gene_name": "Patatin-like phospholipase domain-containing protein 7",
  "gene": "UniProtKB:Q6ZV29"
}